{
  "gene_symbol": "CUL3",
  "term_label": "proteasome-mediated ubiquitin-dependent protein catabolic process",
  "gene": "UniProtKB:Q13618",
  "term_id": "GO:0043161",
  "gene_name": "Cullin-3"
}